core-binding factor complex [GO:0016513] (cellular component) Also known as: CBF complex, AML1 complex, PEPB2 complex Relationships: is a type of RNA polymerase II transcription regulator complex [GO:0090575] References: PMID:15156179, PMID:8497254 Definition: A heterodimeric transcription factor complex that contains an alpha subunit (Runx1, Runx2 or Runx3 in human) that binds DNA and a non-DNA-binding beta subunit (CBFbeta), and binds to a consensus sequence 5'-YGYGGTY-3' found in several enhancers and promoters; the beta subunit enhances the DNA binding of the alpha subunit.